primary miRNA binding [GO:0070878] (molecular function) Also known as: pri-miRNA binding, primary microRNA binding References: PMID:15531877, PMID:15574589 Sources: GOC:sl Definition: Binding to a primary microRNA (pri-miRNA) transcript, an RNA molecule that is processed into a short hairpin-shaped structure called a pre-miRNA and finally into a functional miRNA. Both double-stranded and single-stranded regions of a pri-miRNA are required for binding. Relationships: is a type of RNA binding [GO:0003723]